{
  "gene_name": "Xaa-Pro aminopeptidase 2",
  "gene": "UniProtKB:O43895",
  "gene_symbol": "XPNPEP2",
  "term_id": "UNKNOWN:0001",
  "term_label": "Unknown molecular function"
}